{
  "gene_symbol": "TYK2",
  "gene_name": "Non-receptor tyrosine-protein kinase TYK2",
  "term_label": "non-membrane spanning protein tyrosine kinase activity",
  "term_id": "GO:0004715",
  "gene": "UniProtKB:P29597"
}